{
  "term_label": "olfactory receptor activity",
  "term_id": "GO:0004984",
  "gene_symbol": "OR2C3",
  "gene_name": "Olfactory receptor 2C3",
  "gene": "UniProtKB:Q8N628"
}